{
  "gene_name": "Endothelial cell-specific molecule 1",
  "term_id": "GO:0001525",
  "term_label": "angiogenesis",
  "gene_symbol": "ESM1",
  "gene": "UniProtKB:Q9NQ30"
}